{
  "gene_name": "Guanylyl cyclase-activating protein 3",
  "term_label": "calcium ion binding",
  "gene_symbol": "GUCA1C",
  "term_id": "GO:0005509",
  "gene": "UniProtKB:O95843"
}